tartrate metabolic process [GO:1901275] (BP) Definition: The chemical reactions and pathways involving tartrate. Sources: GOC:TermGenie, GOC:yaf, UniPathway:UPA00839 Also known as: tartrate metabolism Relationships: is a type of metabolic process [GO:0008152] Subtypes: tartrate catabolic process [GO:1901276], tartrate biosynthetic process [GO:1901277]